positive regulation of antimicrobial peptide biosynthetic process [GO:0002807] (biological process) Also known as: up regulation of antimicrobial peptide biosynthetic process, up-regulation of antimicrobial peptide biosynthetic process, upregulation of antimicrobial peptide biosynthetic process, activation of antimicrobial peptide biosynthetic process, stimulation of antimicrobial peptide biosynthetic process Definition: Any process that activates or increases the frequency, rate, or extent of antimicrobial peptide biosynthesis. Subtypes: positive regulation of antibacterial peptide biosynthetic process [GO:0006963], positive regulation of antifungal peptide biosynthetic process [GO:0006967] Relationships: is a type of GO:0002225; is a type of regulation of antimicrobial peptide biosynthetic process [GO:0002805]; positively regulates antimicrobial peptide biosynthetic process [GO:0002777] Sources: GOC:add